regulation of amphiregulin production [GO:0140731] (biological process) Definition: Any process that modulates the frequency, rate, or extent of production of amphiregulin. Relationships: is a type of regulation of cytokine production [GO:0001817]; regulates amphiregulin production [GO:0140730] Subtypes: GO:0140732 References: PMID:24463227 Also known as: regulation of AREG production